cellular response to light intensity [GO:0071484] (biological process) Sources: GOC:mah Subtypes: cellular response to absence of light [GO:0071485], cellular response to high light intensity [GO:0071486], cellular response to low light intensity stimulus [GO:0071487], cellular response to very low light intensity stimulus [GO:0071488] Relationships: is a type of response to light intensity [GO:0009642]; is_a GO:0071482 Definition: Any process that results in a change in state or activity of a cell (in terms of movement, secretion, enzyme production, gene expression, etc.) as a result of a light intensity stimulus.